{
  "term_id": "UNKNOWN:0003",
  "gene_symbol": "SNAI2",
  "term_label": "Unknown cellular component",
  "gene": "UniProtKB:O43623",
  "gene_name": "Zinc finger protein SNAI2"
}